{
  "gene_name": "Src kinase-associated phosphoprotein 2",
  "term_label": "Unknown biological process",
  "gene": "UniProtKB:O75563",
  "term_id": "UNKNOWN:0002",
  "gene_symbol": "SKAP2"
}